regulation of inosine transport [GO:0035341] (biological process) Definition: Any process that modulates the frequency, rate or extent of the directed movement of inosine into, out of or within a cell, or between cells, by means of some agent such as a transporter or pore. Sources: GOC:bf Subtypes: GO:0035342, negative regulation of inosine transport [GO:0035343] Also known as: regulation of hypoxanthine riboside transport Relationships: is a type of regulation of purine nucleoside transport [GO:0032245]; regulates inosine transport [GO:0035340]